{
  "gene": "UniProtKB:Q9BQT9",
  "gene_name": "Calsyntenin-3",
  "gene_symbol": "CLSTN3",
  "term_label": "homophilic cell-cell adhesion",
  "term_id": "GO:0007156"
}